{
  "gene_name": "PRAME family member 20",
  "gene_symbol": "PRAMEF20",
  "term_id": "GO:0043161",
  "gene": "UniProtKB:Q5VT98",
  "term_label": "proteasome-mediated ubiquitin-dependent protein catabolic process"
}